{
  "gene_name": "HLA class II histocompatibility antigen, DM beta chain",
  "gene_symbol": "HLA-DMB",
  "gene": "UniProtKB:P28068",
  "term_label": "MHC class II protein complex",
  "term_id": "GO:0042613"
}